{
  "gene": "UniProtKB:O15480",
  "term_id": "GO:0005634",
  "gene_name": "Melanoma-associated antigen B3",
  "gene_symbol": "MAGEB3",
  "term_label": "nucleus"
}